tRNA modification [GO:0006400] (biological process) Note: The term 'RNA editing' (GO:0016547) was merged into 'RNA modification' (GO:0009451) on the basis of statements in the preface of Modification and Editing of RNA (ISBN:1555811337) that there is no clear distinction between modification and editing. Parallel changes were made for substrate (e.g. tRNA, rRNA, etc.) specific child terms of 'RNA editing'. Also known as: tRNA editing Relationships: is a type of tRNA processing [GO:0008033]; is a type of GO:0009451 Subtypes: tRNA wobble base modification [GO:0002097], archaeosine-tRNA biosynthetic process [GO:0002927], tRNA dihydrouridine synthesis [GO:0002943], tRNA threonylcarbamoyladenosine modification [GO:0002949], GO:0019988, tRNA methylation [GO:0030488], tRNA pseudouridine synthesis [GO:0031119], wybutosine biosynthetic process [GO:0031591], tRNA thio-modification [GO:0034227], tRNA methylthiolation [GO:0035600], GO:0051391, cyclic threonylcarbamoyladenosine biosynthetic process [GO:0061504], tRNA seleno-modification [GO:0070329], GO:0070900, tRNA adenosine deamination to inosine [GO:0140023], GO:1990983 Sources: GOC:curators Definition: The covalent alteration of one or more nucleotides within a tRNA molecule to produce a tRNA molecule with a sequence that differs from that coded genetically.